{
  "gene_symbol": "MPPE1",
  "gene_name": "Metallophosphoesterase 1",
  "gene": "UniProtKB:Q53F39",
  "term_label": "Unknown cellular component",
  "term_id": "UNKNOWN:0003"
}